{
  "gene": "UniProtKB:Q9H2M9",
  "gene_name": "Rab3 GTPase-activating protein non-catalytic subunit",
  "term_label": "establishment of protein localization to endoplasmic reticulum membrane",
  "term_id": "GO:0097051",
  "gene_symbol": "RAB3GAP2"
}